negative regulation of female receptivity, post-mating [GO:0045434] (biological process) Also known as: down regulation of female receptivity, post-mating, down-regulation of female receptivity, post-mating, downregulation of female receptivity, post-mating, inhibition of female receptivity, post-mating Relationships: is a type of GO:0007621; is a type of regulation of female receptivity, post-mating [GO:0046008] References: PMID:11092827 Sources: GOC:bf Definition: Any process that stops, prevents or reduces the receptiveness of a female to male advances subsequent to mating.